{
  "term_label": "Unknown cellular component",
  "term_id": "UNKNOWN:0003",
  "gene": "UniProtKB:Q5W0B7",
  "gene_name": "Transmembrane protein 236",
  "gene_symbol": "TMEM236"
}